phosphatidylinositol-3,4,5-trisphosphate 5-phosphatase activity [GO:0034485] (molecular function) Relationships: is a type of phosphatidylinositol trisphosphate phosphatase activity [GO:0034594]; is_a phosphatidylinositol phosphate 5-phosphatase activity [GO:0034595] Sources: EC:3.1.3.86, GOC:pf Definition: 1,2-diacyl-sn-glycero-3-phospho-(1D-myo-inositol-3,4,5-trisphosphate) + H2O = 1,2-diacyl-sn-glycero-3-phospho-(1D-myo-inositol-3,4-bisphosphate) + phosphate. Regulation: negatively regulated by GO:2001145